glycosome lumen [GO:0034468] (cellular component) Definition: The volume enclosed by the membrane of a glycosome. Sources: GOC:rph Relationships: is a type of GO:0005782; BFO_0000050 glycosome [GO:0020015]